{
  "gene": "UniProtKB:O95497",
  "term_id": "GO:0015939",
  "gene_name": "Pantetheinase",
  "term_label": "pantothenate metabolic process",
  "gene_symbol": "VNN1"
}